glycerol-3-phosphate transmembrane transporter activity [GO:0015169] (molecular function) Relationships: is a type of organophosphate ester transmembrane transporter activity [GO:0015605]; is a type of carbohydrate derivative transmembrane transporter activity [GO:1901505]; is part of glycerol-3-phosphate transmembrane transport [GO:0015794] Subtypes: ABC-type glycerol-3-phosphate transporter activity [GO:0015430] Definition: Enables the transfer of glycerol-3-phosphate from one side of a membrane to the other. Glycerol-3-phosphate is a phosphoric monoester of glycerol. Sources: GOC:ai